{
  "gene_name": "Adenosylhomocysteinase 3",
  "gene_symbol": "AHCYL2",
  "term_id": "UNKNOWN:0001",
  "term_label": "Unknown molecular function",
  "gene": "UniProtKB:Q96HN2"
}